 [go#goslim:yeast] Note: Yeast GO slim